{
  "term_label": "plasma membrane",
  "gene": "UniProtKB:Q9BXB1",
  "term_id": "GO:0005886",
  "gene_name": "Leucine-rich repeat-containing G-protein coupled receptor 4",
  "gene_symbol": "LGR4"
}